{
  "term_label": "intracellular signal transduction",
  "term_id": "GO:0035556",
  "gene": "UniProtKB:Q8IWV1",
  "gene_name": "Lymphocyte transmembrane adapter 1",
  "gene_symbol": "LAX1"
}